pallium glioblast division [GO:0022016] (biological process) Relationships: is a type of GO:0048860; is part of pallium cell proliferation in forebrain [GO:0022013] Also known as: glioblast cell division in pallium Definition: The division of a glioblast in the pallium. A glioblast is a dividing precursor cell that gives rise to glial cells. Sources: GOC:cls, GOC:dgh, GOC:dph, GOC:jid, GO_REF:0000021